DNA deamination [GO:0045006] (biological process) Subtypes: DNA cytosine deamination [GO:0070383] Sources: GOC:ai Definition: The removal of an amino group from a nucleotide base in DNA. An example is the deamination of cytosine to produce uracil. Relationships: is a type of DNA modification [GO:0006304]